{
  "term_label": "Unknown cellular component",
  "gene": "UniProtKB:O14832",
  "gene_name": "Phytanoyl-CoA dioxygenase, peroxisomal",
  "term_id": "UNKNOWN:0003",
  "gene_symbol": "PHYH"
}